{
  "gene_symbol": "OR7C1",
  "gene": "UniProtKB:O76099",
  "term_id": "GO:0004984",
  "gene_name": "Olfactory receptor 7C1",
  "term_label": "olfactory receptor activity"
}